{
  "term_id": "UNKNOWN:0002",
  "gene_symbol": "CLCA2",
  "gene": "UniProtKB:Q9UQC9",
  "gene_name": "Calcium-activated chloride channel regulator 2",
  "term_label": "Unknown biological process"
}